ceramide binding [GO:0097001] (molecular function) Relationships: is a type of GO:0033218; is a type of GO:0046625 Definition: Binding to a ceramide, a class of lipids composed of sphingosine linked to a fatty acid. Ceramides are a major component of cell membranes. Subtypes: ganglioside binding [GO:0035594], ceramide 1-phosphate binding [GO:1902387] Sources: GOC:sart